{
  "gene": "UniProtKB:P61289",
  "gene_symbol": "PSME3",
  "term_label": "regulation of proteasomal protein catabolic process",
  "gene_name": "Proteasome activator complex subunit 3",
  "term_id": "GO:0061136"
}